{
  "term_label": "Unknown molecular function",
  "term_id": "UNKNOWN:0001",
  "gene": "UniProtKB:Q16799",
  "gene_symbol": "RTN1",
  "gene_name": "Reticulon-1"
}